{
  "gene_symbol": "RTTN",
  "term_label": "ciliary basal body",
  "term_id": "GO:0036064",
  "gene_name": "Rotatin",
  "gene": "UniProtKB:Q86VV8"
}